{
  "term_id": "GO:0007166",
  "gene_symbol": "C17orf99",
  "gene": "UniProtKB:Q6UX52",
  "gene_name": "Protein IL-40",
  "term_label": "cell surface receptor signaling pathway"
}